{
  "term_id": "GO:0005102",
  "gene": "UniProtKB:Q6UWQ7",
  "gene_symbol": "IGFL2",
  "term_label": "signaling receptor binding",
  "gene_name": "Insulin growth factor-like family member 2"
}